subnuclear spatial organization of silent mating-type cassette heterochromatin [GO:0140464] (biological process) References: PMID:26744419 Also known as: silent mating-type cassette heterochromatin spatial organization in the nucleus, silent mating-type cassette heterochromatin organization Definition: The localization of silent mating-type cassette heterochromatin at a specific location in the nucleus. Relationships: is a type of chromosome attachment to the nuclear envelope [GO:0097240]